{
  "gene": "UniProtKB:A0A0C4DH29",
  "gene_name": "Immunoglobulin heavy variable 1-3",
  "term_label": "antigen binding",
  "term_id": "GO:0003823",
  "gene_symbol": "IGHV1-3"
}